regulation of oxidative stress-induced intrinsic apoptotic signaling pathway [GO:1902175] (biological process) Subtypes: negative regulation of oxidative stress-induced intrinsic apoptotic signaling pathway [GO:1902176], GO:1902177, regulation of oxidative stress-induced neuron intrinsic apoptotic signaling pathway [GO:1903376], regulation of intrinsic apoptotic signaling pathway in response to hydrogen peroxide [GO:1903750] Definition: Any process that modulates the frequency, rate or extent of an oxidative stress-induced intrinsic apoptotic signaling pathway. Also known as: regulation of intrinsic apoptotic signaling pathway in response to oxidative stress Relationships: is a type of regulation of intrinsic apoptotic signaling pathway [GO:2001242]; regulates intrinsic apoptotic signaling pathway in response to oxidative stress [GO:0008631] References: PMID:11672522 Sources: GOC:BHF, GOC:TermGenie, GOC:mtg_apoptosis